thylakoid lumen [GO:0031977] (cellular component) Sources: GOC:mah, GOC:pz Relationships: is a type of cellular anatomical structure [GO:0110165]; is part of GO:0009579 Definition: The volume enclosed by a thylakoid membrane. Subtypes: plastid thylakoid lumen [GO:0031978], plasma membrane-derived thylakoid lumen [GO:0031979], GO:0070117